2-hydroxyisocaproate CoA-transferase activity [GO:0043712] (molecular function) References: PMID:16957230 Relationships: is a type of GO:0008410 Definition: Catalysis of the reaction: (R)-2-hydroxyisocaproate + isocaproyl-CoA = (R)-2-hydroxyisocaproyl-CoA + isocaproate. Also known as: (R)-2-hydroxyisocaproate CoA transferase activity, (R)-2-hydroxyisocaproate CoA-transferase activity